synergid death [GO:0010198] (biological process) Relationships: is a type of developmental process involved in reproduction [GO:0003006]; is a type of GO:0010623; is part of pollination [GO:0009856] Definition: Synergid cells undergo degeneration and death in response to penetration by the pollen tube. It is an active process that involves a dramatic decrease in cell volume, collapse of the vacuoles, and complete disintegration of the plasma membrane and most organelles. Also known as: synergid cell death, synergid degeneration References: PMID:12215516 Sources: GOC:isa_complete, GOC:sm